negative regulation of peptidyl-cysteine S-nitrosylation [GO:1902083] (biological process) Definition: Any process that stops, prevents or reduces the frequency, rate or extent of peptidyl-cysteine S-nitrosylation. References: PMID:19198614 Sources: GOC:BHF, GOC:TermGenie, GOC:rl Also known as: down regulation of S-nitrosylation, down regulation of peptidyl-cysteine S-nitrosylation, down regulation of protein S-nitrosylation, down-regulation of S-nitrosylation, down-regulation of peptidyl-cysteine S-nitrosylation, down-regulation of protein S-nitrosylation, downregulation of S-nitrosylation, downregulation of peptidyl-cysteine S-nitrosylation, downregulation of protein S-nitrosylation, inhibition of S-nitrosylation, inhibition of protein S-nitrosylation, negative regulation of S-nitrosylation, negative regulation of protein S-nitrosylation, inhibition of peptidyl-cysteine S-nitrosylation Relationships: is a type of negative regulation of protein modification process [GO:0031400]; is a type of regulation of peptidyl-cysteine S-nitrosylation [GO:2000169]; RO_0002212 peptidyl-cysteine S-nitrosylation [GO:0018119]